{
  "gene_symbol": "LZTR1",
  "term_label": "Golgi apparatus",
  "gene_name": "Leucine-zipper-like transcriptional regulator 1",
  "term_id": "GO:0005794",
  "gene": "UniProtKB:Q8N653"
}